{
  "gene_symbol": "G2E3",
  "term_label": "Unknown biological process",
  "term_id": "UNKNOWN:0002",
  "gene": "UniProtKB:Q7L622",
  "gene_name": "G2_M phase-specific E3 ubiquitin-protein ligase"
}